{
  "term_label": "collagen fibril organization",
  "term_id": "GO:0030199",
  "gene": "UniProtKB:O60568",
  "gene_symbol": "PLOD3",
  "gene_name": "Multifunctional procollagen lysine hydroxylase and glycosyltransferase LH3"
}